{
  "gene": "UniProtKB:Q460N5",
  "term_label": "transcription corepressor activity",
  "gene_symbol": "PARP14",
  "gene_name": "Protein mono-ADP-ribosyltransferase PARP14",
  "term_id": "GO:0003714"
}